{
  "gene": "UniProtKB:A0A0U1RRN3",
  "gene_symbol": "MISFA",
  "term_label": "Unknown cellular component",
  "gene_name": "Mitochondrial sheath formation-associated protein",
  "term_id": "UNKNOWN:0003"
}